{
  "gene": "UniProtKB:O75385",
  "term_label": "cytosol",
  "term_id": "GO:0005829",
  "gene_symbol": "ULK1",
  "gene_name": "Serine_threonine-protein kinase ULK1"
}